{
  "gene": "UniProtKB:Q9ULD2",
  "gene_name": "Microtubule-associated tumor suppressor 1",
  "gene_symbol": "MTUS1",
  "term_label": "nucleus",
  "term_id": "GO:0005634"
}